{
  "gene": "UniProtKB:Q63ZY6",
  "term_label": "Unknown biological process",
  "gene_name": "Putative methyltransferase NSUN5C",
  "term_id": "UNKNOWN:0002",
  "gene_symbol": "NSUN5P2"
}